{
  "gene_name": "F-box only protein 16",
  "gene_symbol": "FBXO16",
  "term_label": "Unknown molecular function",
  "gene": "UniProtKB:Q8IX29",
  "term_id": "UNKNOWN:0001"
}